{
  "term_id": "GO:0003727",
  "term_label": "single-stranded RNA binding",
  "gene_name": "Antiviral innate immune response receptor RIG-I",
  "gene": "UniProtKB:O95786",
  "gene_symbol": "RIGI"
}